mycothiol biosynthetic process [GO:0010125] (biological process) Relationships: is a type of GO:0010126; is a type of glycoside biosynthetic process [GO:0016138]; is a type of sulfur compound biosynthetic process [GO:0044272] Also known as: mycothiol anabolism, mycothiol biosynthesis, mycothiol formation, mycothiol synthesis Sources: GOC:pz Definition: The chemical reactions and pathways resulting in the formation of mycothiol, which consists of N-acetyl-L-cysteine linked to a pseudodisaccharide, D-glucosamine and myo-inositol. Mycothiol is produced in actinomycetes like mycobacteria and serves similar functions to glutathione.